{
  "term_label": "Unknown cellular component",
  "gene_name": "PALM2 and AKAP2 fusion",
  "gene_symbol": "PALM2AKAP2",
  "term_id": "UNKNOWN:0003",
  "gene": "UniProtKB:C9JA33"
}